beta selection [GO:0043366] (biological process) Definition: The process in which successful recombination of a T cell receptor beta chain into a translatable protein coding sequence leads to rescue from apoptosis and subsequent proliferation of an immature T cell. References: PMID:12220932 Sources: ISBN:0781735149 Relationships: is_a T cell selection [GO:0045058]; is part of alpha-beta T cell differentiation [GO:0046632]